{
  "term_id": "GO:0016491",
  "gene_symbol": "DHRS9",
  "gene": "UniProtKB:Q9BPW9",
  "term_label": "oxidoreductase activity",
  "gene_name": "Dehydrogenase_reductase SDR family member 9"
}